{
  "gene_name": "Fibroblast growth factor-binding protein 3",
  "term_id": "UNKNOWN:0003",
  "term_label": "Unknown cellular component",
  "gene_symbol": "FGFBP3",
  "gene": "UniProtKB:Q8TAT2"
}